{
  "term_label": "Unknown cellular component",
  "gene": "UniProtKB:Q495D7",
  "term_id": "UNKNOWN:0003",
  "gene_symbol": "LINC01559",
  "gene_name": "Putative uncharacterized protein encoded by LINC01559"
}